{
  "term_label": "regulation of transcription by RNA polymerase II",
  "gene_symbol": "GCM2",
  "gene": "UniProtKB:O75603",
  "gene_name": "Chorion-specific transcription factor GCMb",
  "term_id": "GO:0006357"
}